{
  "term_label": "secretory granule",
  "gene_name": "Oxytocin-neurophysin 1",
  "gene": "UniProtKB:P01178",
  "gene_symbol": "OXT",
  "term_id": "GO:0030141"
}